{
  "gene_name": "Cerebellar degeneration-related protein 2",
  "gene": "UniProtKB:Q01850",
  "term_label": "Unknown biological process",
  "gene_symbol": "CDR2",
  "term_id": "UNKNOWN:0002"
}